hematopoietic stem cell differentiation [GO:0060218] (biological process) References: PMID:15378083 Sources: GOC:BHF, GOC:bf, GOC:dph, GOC:rl Also known as: haematopoietic stem cell differentiation, haemopoietic stem cell differentiation, hemopoietic stem cell differentiation Relationships: is a type of hematopoietic progenitor cell differentiation [GO:0002244]; is a type of GO:0048863 Definition: The process in which a relatively unspecialized cell acquires specialized features of a hematopoietic stem cell. A stem cell is a cell that retains the ability to divide and proliferate throughout life to provide progenitor cells that can differentiate into specialized cells. Regulation: regulated by regulation of hematopoietic stem cell differentiation [GO:1902036]; negatively regulated by negative regulation of hematopoietic stem cell differentiation [GO:1902037]; positively regulated by positive regulation of hematopoietic stem cell differentiation [GO:1902038]